{
  "term_label": "cytoplasm",
  "gene_name": "Calcineurin B homologous protein 3",
  "term_id": "GO:0005737",
  "gene": "UniProtKB:Q96BS2",
  "gene_symbol": "TESC"
}